{
  "gene_name": "Myelin-associated neurite-outgrowth inhibitor",
  "term_id": "UNKNOWN:0002",
  "gene_symbol": "FAM168B",
  "term_label": "Unknown biological process",
  "gene": "UniProtKB:A1KXE4"
}